16S rRNA (guanine(966)-N(2))-methyltransferase activity [GO:0052913] (molecular function) Definition: Catalysis of the reaction: S-adenosyl-L-methionine + guanosine(966) in 16S rRNA = N(2)-methylguanosine(966) in 16S rRNA + S-adenosyl-L-homocysteine. Relationships: is a type of rRNA (guanine-N2-)-methyltransferase activity [GO:0008990] Sources: EC:2.1.1.171